{
  "gene": "UniProtKB:Q6ZV80",
  "term_id": "UNKNOWN:0001",
  "gene_symbol": "LINC02898",
  "term_label": "Unknown molecular function",
  "gene_name": "Putative uncharacterized protein LINC02898"
}